{
  "gene_symbol": "MMAB",
  "gene": "UniProtKB:Q96EY8",
  "term_id": "UNKNOWN:0002",
  "gene_name": "Corrinoid adenosyltransferase MMAB",
  "term_label": "Unknown biological process"
}